{
  "term_id": "GO:0006357",
  "gene_symbol": "ZNF551",
  "gene_name": "Zinc finger protein 551",
  "gene": "UniProtKB:Q7Z340",
  "term_label": "regulation of transcription by RNA polymerase II"
}